specification of symmetry [GO:0009799] (biological process) Subtypes: determination of bilateral symmetry [GO:0009855], GO:0009879, specification of ureteric bud anterior/posterior symmetry [GO:0072100] Relationships: is_a pattern specification process [GO:0007389] Also known as: determination of symmetry Definition: The establishment of an organism's body plan or part of an organism such that a similar arrangement in form and relationship of parts around a common axis, or around each side of a plane is created. Sources: GOC:go_curators